{
  "gene": "UniProtKB:Q5T1M5",
  "gene_symbol": "FKBP15",
  "gene_name": "FK506-binding protein 15",
  "term_id": "UNKNOWN:0002",
  "term_label": "Unknown biological process"
}